{
  "gene_name": "Pyruvate dehydrogenase protein X component, mitochondrial",
  "gene_symbol": "PDHX",
  "term_id": "GO:0005739",
  "term_label": "mitochondrion",
  "gene": "UniProtKB:O00330"
}